{
  "gene_name": "Amyloid-beta A4 precursor protein-binding family A member 2",
  "gene": "UniProtKB:Q99767",
  "term_label": "cytoplasm",
  "term_id": "GO:0005737",
  "gene_symbol": "APBA2"
}